{
  "gene_symbol": "PHGDH",
  "gene_name": "D-3-phosphoglycerate dehydrogenase",
  "term_id": "UNKNOWN:0002",
  "term_label": "Unknown biological process",
  "gene": "UniProtKB:O43175"
}